activation of adenylate cyclase activity [GO:0007190] (biological process) Definition: Any process that initiates the activity of the inactive enzyme adenylate cyclase. Relationships: is a type of positive regulation of adenylate cyclase activity [GO:0045762] Sources: GOC:ai Also known as: adenylate cyclase activation, adenylyl cyclase activation, adenylate cyclase activator